{
  "gene_name": "Polycystin-1-like protein 3",
  "term_id": "GO:0016020",
  "term_label": "membrane",
  "gene": "UniProtKB:Q7Z443",
  "gene_symbol": "PKD1L3"
}